{
  "term_label": "G protein-coupled receptor activity",
  "gene_name": "G-protein coupled receptor 15",
  "term_id": "GO:0004930",
  "gene": "UniProtKB:P49685",
  "gene_symbol": "GPR15"
}